{
  "term_id": "GO:0042254",
  "gene": "UniProtKB:Q96HR8",
  "gene_name": "H_ACA ribonucleoprotein complex non-core subunit NAF1",
  "term_label": "ribosome biogenesis",
  "gene_symbol": "NAF1"
}